cyclic GMP-AMP synthase activity [GO:0140699] (molecular function) Note: Note that this term should not be used for direct annotation. It should be possible to annotate to a more specific child term that describes the position of the phosphate group on the cGAMP molecule. Also known as: cyclic-GMP-AMP synthase activity Subtypes: 2',3'-cyclic GMP-AMP synthase activity [GO:0061501], GO:0140700, 3',3'-cyclic GMP-AMP synthase activity [GO:0140701] Relationships: is a type of nucleotidyltransferase activity [GO:0016779] Definition: Catalysis of the reaction: ATP + GTP = 2 diphosphate + cyclic GMP-AMP. References: PMID:23258413